{
  "gene": "UniProtKB:Q15063",
  "gene_symbol": "POSTN",
  "gene_name": "Periostin",
  "term_label": "cell adhesion",
  "term_id": "GO:0007155"
}